{
  "term_label": "Unknown biological process",
  "gene": "UniProtKB:A6NEL2",
  "gene_name": "Ankyrin repeat domain-containing protein SOWAHB",
  "gene_symbol": "SOWAHB",
  "term_id": "UNKNOWN:0002"
}